prephenate dehydratase activity [GO:0004664] (MF) Definition: Catalysis of the reaction: prephenate = phenylpyruvate + H2O + CO2. Sources: EC:4.2.1.51 Relationships: is a type of hydro-lyase activity [GO:0016836] Also known as: prephenate hydro-lyase (decarboxylating), prephenate hydro-lyase (decarboxylating; phenylpyruvate-forming)